plant-type secondary cell wall biogenesis [GO:0009834] (biological process) Relationships: is a type of GO:0009832 Regulation: negatively regulated by GO:1901347; positively regulated by positive regulation of secondary cell wall biogenesis [GO:1901348]; regulated by GO:2000652 Definition: A cellular process that results in the biosynthesis of constituent macromolecules, assembly, and arrangement of constituent parts of inextensible cellulose- and pectin-containing cell walls that are formed between the plasma membrane and primary cell wall after cell expansion is complete. An example of this is found in Arabidopsis thaliana. Sources: GOC:lr, GOC:mtg_sensu Subtypes: GO:0090379 Also known as: secondary cell wall anabolism, secondary cell wall biosynthetic process, secondary cell wall formation, secondary cell wall synthesis, cellulose and pectin-containing secondary cell wall biogenesis, secondary cell wall biogenesis